proximal dendrite [GO:1990635] (cellular component) References: PMID:16899232 Sources: GOC:aruk, GOC:bc Relationships: is a type of dendrite [GO:0030425] Definition: The dendrite of the dendritic tree that is closest to the neuronal cell body (the soma). Subtypes: apical proximal dendrite [GO:0150015], GO:0150017